endoderm formation [GO:0001706] (biological process) Relationships: is a type of formation of primary germ layer [GO:0001704]; is part of endoderm development [GO:0007492] Sources: GOC:go_curators Definition: The formation of the endoderm during gastrulation. Also known as: endoblast formation